spindle attachment to meiosis I kinetochore [GO:0051455] (BP) Definition: The cellular process in which spindle microtubules become physically associated with the proteins making up the kinetochore complex in meiosis I. During meiosis I sister kinetochores are lying next to each other facing the same spindle pole and monopolar attachment of the chromatid to the spindle occurs. Regulation: regulated by regulation of spindle attachment to meiosis I kinetochore [GO:1904967]; positively regulated by positive regulation of spindle attachment to meiosis I kinetochore [GO:1904968] Also known as: attachment of spindle microtubules to kinetochore involved in homologous chromosome segregation, attachment of spindle microtubules to kinetochore involved in meiosis I, attachment of spindle microtubules to kinetochore during meiosis I, monopolar attachment, sister kinetochore mono-orientation Sources: GOC:ai, GOC:clt, GOC:dph, GOC:tb Relationships: is a type of attachment of meiotic spindle microtubules to kinetochore [GO:0051316]; is part of meiotic metaphase I homologous chromosome alignment [GO:0043060] Note: Note that the synonym 'monopolar attachment' refers to the normal attachment of sister chromosomes to the spindle in meiosis I, and not to the aberrant attachment of sister kinetochores to a single pole in mitosis.